3-methylbut-2-enoyl-CoA(4-) metabolic process [GO:1902198] (biological process) References: PMID:11231285 Sources: GOC:TermGenie Relationships: is_a GO:0035337 Definition: The chemical reactions and pathways involving 3-methylbut-2-enoyl-CoA(4-). Also known as: 3-methylbut-2-enoyl-CoA(4-) metabolism Subtypes: 3-methylbut-2-enoyl-CoA(4-) catabolic process [GO:1902199], 3-methylbut-2-enoyl-CoA(4-) biosynthetic process [GO:1902200]